{
  "gene_symbol": "TOX3",
  "term_id": "GO:0006357",
  "gene": "UniProtKB:O15405",
  "term_label": "regulation of transcription by RNA polymerase II",
  "gene_name": "TOX high mobility group box family member 3"
}